{
  "gene": "UniProtKB:P08138",
  "term_label": "nerve growth factor binding",
  "gene_name": "Tumor necrosis factor receptor superfamily member 16",
  "term_id": "GO:0048406",
  "gene_symbol": "NGFR"
}